{
  "gene_symbol": "USP17L18",
  "term_id": "GO:0005634",
  "gene_name": "Ubiquitin carboxyl-terminal hydrolase 17-like protein 18",
  "gene": "UniProtKB:D6R9N7",
  "term_label": "nucleus"
}